{
  "gene": "UniProtKB:Q96AK3",
  "gene_name": "DNA dC-dU-editing enzyme APOBEC-3D",
  "gene_symbol": "APOBEC3D",
  "term_label": "cytoplasm",
  "term_id": "GO:0005737"
}